{
  "gene": "UniProtKB:Q9H920",
  "term_label": "Golgi membrane",
  "gene_symbol": "RNF121",
  "term_id": "GO:0000139",
  "gene_name": "E3 ubiquitin ligase RNF121"
}